{
  "term_label": "DNA-binding transcription factor activity, RNA polymerase II-specific",
  "gene": "UniProtKB:P0DPD5",
  "term_id": "GO:0000981",
  "gene_symbol": "ZNF723",
  "gene_name": "Zinc finger protein 723"
}